regulation of intraciliary anterograde transport [GO:1905796] (biological process) References: PMID:27930654 Sources: GOC:TermGenie, GO_REF:0000058 Also known as: regulation of intraflagellar anterograde transport Definition: Any process that modulates the frequency, rate or extent of intraciliary anterograde transport. Subtypes: negative regulation of intraciliary anterograde transport [GO:1905797], positive regulation of intraciliary anterograde transport [GO:1905798] Relationships: is a type of regulation of intracellular transport [GO:0032386]; is a type of GO:0060632; regulates intraciliary anterograde transport [GO:0035720]